{
  "gene": "UniProtKB:Q16650",
  "term_label": "regulation of transcription by RNA polymerase II",
  "gene_symbol": "TBR1",
  "term_id": "GO:0006357",
  "gene_name": "T-box brain protein 1"
}